{
  "gene_name": "Pleckstrin homology-like domain family A member 1",
  "gene_symbol": "PHLDA1",
  "term_label": "Unknown molecular function",
  "term_id": "UNKNOWN:0001",
  "gene": "UniProtKB:Q8WV24"
}